N6-methyl-(d)ATP hydrolase activity [GO:0106431] (molecular function) Definition: Catalysis of the reaction N6-methyl-(d)ATP + H2O = N6-methyl-(d)AMP + diphosphate + H+. Relationships: is a type of hydrolase activity, acting on acid anhydrides, in phosphorus-containing anhydrides [GO:0016818] References: PMID:32144205